{
  "gene_symbol": "ATXN1L",
  "gene_name": "Ataxin-1-like",
  "term_id": "GO:0007420",
  "term_label": "brain development",
  "gene": "UniProtKB:P0C7T5"
}